{
  "gene_symbol": "PTH2R",
  "gene_name": "Parathyroid hormone 2 receptor",
  "term_id": "GO:0004991",
  "term_label": "parathyroid hormone receptor activity",
  "gene": "UniProtKB:P49190"
}